{
  "gene": "UniProtKB:P10451",
  "term_id": "GO:0050840",
  "gene_name": "Osteopontin",
  "gene_symbol": "SPP1",
  "term_label": "extracellular matrix binding"
}